{
  "term_id": "GO:0031941",
  "gene": "UniProtKB:Q2TBC4",
  "gene_symbol": "PRICKLE4",
  "gene_name": "Prickle-like protein 4",
  "term_label": "filamentous actin"
}